{
  "term_id": "GO:0002323",
  "gene_symbol": "IFNA8",
  "gene": "UniProtKB:P32881",
  "term_label": "natural killer cell activation involved in immune response",
  "gene_name": "Interferon alpha-8"
}